{
  "gene_name": "Zinc finger protein 564",
  "term_label": "Unknown cellular component",
  "gene_symbol": "ZNF564",
  "gene": "UniProtKB:Q8TBZ8",
  "term_id": "UNKNOWN:0003"
}